{
  "gene_name": "cAMP-dependent protein kinase inhibitor alpha",
  "gene": "UniProtKB:P61925",
  "term_label": "cytoplasm",
  "term_id": "GO:0005737",
  "gene_symbol": "PKIA"
}